{
  "term_label": "nucleus",
  "gene_symbol": "CDK10",
  "gene_name": "Cyclin-dependent kinase 10",
  "term_id": "GO:0005634",
  "gene": "UniProtKB:Q15131"
}